negative regulation of iron ion transport [GO:0034757] (biological process) Subtypes: negative regulation of iron ion transmembrane transport [GO:0034760] Definition: Any process that stops, prevents, or reduces the frequency, rate or extent of the directed movement of iron ions into, out of or within a cell, or between cells, by means of some agent such as a transporter or pore. Relationships: is a type of regulation of iron ion transport [GO:0034756]; is a type of negative regulation of monoatomic ion transport [GO:0043271]; negatively regulates iron ion transport [GO:0006826] Also known as: down regulation of iron ion transport, down-regulation of iron ion transport, downregulation of iron ion transport, negative regulation of iron transport, inhibition of iron ion transport Sources: GOC:mah